{
  "term_id": "UNKNOWN:0002",
  "gene_name": "T-cell immunomodulatory protein",
  "term_label": "Unknown biological process",
  "gene": "UniProtKB:Q8TB96",
  "gene_symbol": "ITFG1"
}